{
  "gene": "UniProtKB:A0A1B0GUY1",
  "term_id": "UNKNOWN:0002",
  "gene_symbol": "MARCOL",
  "term_label": "Unknown biological process",
  "gene_name": "MARCO-like protein"
}